{
  "gene_symbol": "BAGE3",
  "term_label": "Unknown molecular function",
  "gene": "UniProtKB:Q86Y29",
  "gene_name": "B melanoma antigen 3",
  "term_id": "UNKNOWN:0001"
}